negative regulation of cytoplasmic translational elongation through polyproline stretches [GO:1903271] (biological process) Relationships: is a type of negative regulation of cytoplasmic translational elongation [GO:1900248]; is a type of regulation of cytoplasmic translational elongation through polyproline stretches [GO:1903270]; negatively regulates cytoplasmic translational elongation through polyproline stretches [GO:0097622] Definition: Any process that stops, prevents or reduces the frequency, rate or extent of cytoplasmic translational elongation through polyproline stretches. References: PMID:24923804 Sources: GOC:TermGenie, GO_REF:0000058 Also known as: down regulation of cytoplasmic translational elongation through polyproline stretches, down-regulation of cytoplasmic translational elongation through polyproline stretches, downregulation of cytoplasmic translational elongation through polyproline stretches, inhibition of cytoplasmic translational elongation through polyproline stretches